{
  "gene_name": "Beta-microseminoprotein",
  "term_id": "UNKNOWN:0003",
  "term_label": "Unknown cellular component",
  "gene_symbol": "MSMB",
  "gene": "UniProtKB:P08118"
}